{
  "term_id": "GO:0005634",
  "gene": "UniProtKB:A6NFH5",
  "term_label": "nucleus",
  "gene_symbol": "FABP12",
  "gene_name": "Fatty acid-binding protein 12"
}